carpel formation [GO:0048462] (biological process) Sources: GOC:jid Definition: The process that gives rise to the carpel. This process pertains to the initial formation of a structure from unspecified parts. Relationships: is a type of GO:0048449; is part of carpel morphogenesis [GO:0048445]